{
  "gene_symbol": "NFS1",
  "term_label": "cytosol",
  "gene": "UniProtKB:Q9Y697",
  "gene_name": "Cysteine desulfurase",
  "term_id": "GO:0005829"
}